{
  "term_id": "GO:0005739",
  "gene": "UniProtKB:Q96RP9",
  "term_label": "mitochondrion",
  "gene_symbol": "GFM1",
  "gene_name": "Elongation factor G, mitochondrial"
}